{
  "term_label": "Unknown molecular function",
  "gene_name": "Inactive Rho GTPase-activating protein 11B",
  "gene": "UniProtKB:Q3KRB8",
  "term_id": "UNKNOWN:0001",
  "gene_symbol": "ARHGAP11B"
}